{
  "term_id": "GO:0006955",
  "gene_symbol": "IGLV4-3",
  "gene_name": "Immunoglobulin lambda variable 4-3",
  "term_label": "immune response",
  "gene": "UniProtKB:A0A075B6K6"
}